{
  "gene_name": "Leucine-rich repeat-containing protein 7",
  "gene_symbol": "LRRC7",
  "term_id": "GO:0016323",
  "gene": "UniProtKB:Q96NW7",
  "term_label": "basolateral plasma membrane"
}